{
  "term_label": "histone binding",
  "gene_name": "Coordinator of PRMT5 and differentiation stimulator",
  "term_id": "GO:0042393",
  "gene": "UniProtKB:Q9NQ92",
  "gene_symbol": "COPRS"
}